{
  "gene": "UniProtKB:A0A075B7F0",
  "term_id": "GO:0016064",
  "term_label": "immunoglobulin mediated immune response",
  "gene_name": "Immunoglobulin heavy variable 3_OR16-10 (non-functional) (Fragment)",
  "gene_symbol": "IGHV3OR16-10"
}